{
  "term_id": "GO:0031594",
  "gene": "UniProtKB:O94868",
  "gene_symbol": "FCHSD2",
  "term_label": "neuromuscular junction",
  "gene_name": "F-BAR and double SH3 domains protein 2"
}